{
  "term_id": "GO:0071222",
  "gene": "UniProtKB:Q9NZH7",
  "gene_name": "Interleukin-36 beta",
  "term_label": "cellular response to lipopolysaccharide",
  "gene_symbol": "IL36B"
}